{
  "gene_name": "Mitochondrial carrier homolog 1",
  "term_id": "GO:0043065",
  "gene_symbol": "MTCH1",
  "term_label": "positive regulation of apoptotic process",
  "gene": "UniProtKB:Q9NZJ7"
}